mitochondrial large ribosomal subunit binding [GO:0140978] (molecular function) References: PMID:28892042 Relationships: is a type of ribosomal large subunit binding [GO:0043023]; is a type of mitochondrial ribosome binding [GO:0097177] Definition: Binding to a mitochondrial large ribosomal subunit. Also known as: mitochondrial ribosomal large subunit binding